T-helper 1 cell activation [GO:0035711] (biological process) Definition: The change in morphology and behavior of a T-helper 1 cell resulting from exposure to a mitogen, cytokine, chemokine, cellular ligand, or an antigen for which it is specific. Sources: CL:0000545, GOC:BHF Also known as: Th1 cell activation Relationships: is a type of GO:0035710 Regulation: RO_0002211 by regulation of T-helper 1 cell activation [GO:2000517]; negatively regulated by negative regulation of T-helper 1 cell activation [GO:2000518]; positively regulated by positive regulation of T-helper 1 cell activation [GO:2000519]